translation factor activity, RNA binding [GO:0008135] (molecular function) Definition: Functions during translation by binding to RNA during polypeptide synthesis at the ribosome. Sources: GOC:ai, GOC:vw Also known as: translation factor activity, nucleic acid binding Relationships: is a type of translation factor activity [GO:0180051]; BFO_0000050 translation [GO:0006412]; has part GO:0003723